{
  "gene_name": "Angiopoietin-related protein 1",
  "gene": "UniProtKB:O95841",
  "term_label": "extracellular matrix",
  "term_id": "GO:0031012",
  "gene_symbol": "ANGPTL1"
}